{
  "gene_name": "Magnesium transporter MRS2 homolog, mitochondrial",
  "gene": "UniProtKB:Q9HD23",
  "term_label": "mitochondrial magnesium ion transmembrane transport",
  "gene_symbol": "MRS2",
  "term_id": "GO:0045016"
}